response to amylopectin [GO:0044591] (biological process) Sources: GOC:mengo_curators, GOC:tt Definition: A process that results in a change in state or activity of a cell (in terms of movement, secretion, enzyme production, gene expression, etc.) as a result of amylopectin stimulus. Regulation: regulated by GO:1900521; negatively regulated by negative regulation of response to amylopectin [GO:1900522]; RO_0002213 by positive regulation of response to amylopectin [GO:1900523] Relationships: is a type of response to oxygen-containing compound [GO:1901700]